tetracycline transmembrane transporter activity [GO:0008493] (molecular function) Also known as: tetracyclin transporter activity, tetracycline transporter activity Sources: GOC:curators Subtypes: tetracycline:proton antiporter activity [GO:0015520] Definition: Enables the transfer of tetracycline from one side of a membrane to the other. Tetracycline is a broad spectrum antibiotic that blocks binding of aminoacyl tRNA to the ribosomes of both Gram-positive and Gram-negative organisms (and those of organelles). Relationships: is a type of GO:0015665; is part of tetracycline transmembrane transport [GO:0015904]